{
  "gene_symbol": "POP7",
  "gene_name": "Ribonuclease P protein subunit p20",
  "gene": "UniProtKB:O75817",
  "term_label": "nucleus",
  "term_id": "GO:0005634"
}